{
  "gene": "UniProtKB:Q9H706",
  "gene_symbol": "GAREM1",
  "term_label": "epidermal growth factor receptor signaling pathway",
  "gene_name": "GRB2-associated and regulator of MAPK protein 1",
  "term_id": "GO:0007173"
}